pancreatic bud formation [GO:0061130] (biological process) Definition: The morphogenetic process in which the foregut region specified to become the pancreas forms a bud. Sources: GOC:dph Relationships: is a type of animal organ formation [GO:0048645]; is a type of branching involved in pancreas morphogenesis [GO:0061114]; is_a epithelial tube formation [GO:0072175]